{
  "gene": "UniProtKB:Q8NHY3",
  "term_id": "GO:0031110",
  "gene_name": "GAS2-like protein 2",
  "gene_symbol": "GAS2L2",
  "term_label": "regulation of microtubule polymerization or depolymerization"
}